3-sulfino-L-alanine binding [GO:0036127] (molecular function) Definition: Binding to 3-sulfino-L-alanine (cysteine sulfinate). Also known as: cysteine sulfinate binding References: PMID:8346915 Sources: GOC:al Relationships: is a type of GO:0016597; is a type of carboxylic acid binding [GO:0031406]; is a type of modified amino acid binding [GO:0072341]; is a type of sulfur compound binding [GO:1901681]